{
  "gene": "UniProtKB:Q99807",
  "gene_name": "5-demethoxyubiquinone hydroxylase, mitochondrial",
  "gene_symbol": "COQ7",
  "term_id": "GO:0006744",
  "term_label": "ubiquinone biosynthetic process"
}